cellular response to inositol [GO:1902141] (biological process) Relationships: is a type of cellular response to oxygen-containing compound [GO:1901701]; is a type of response to inositol [GO:1902140] Definition: Any process that results in a change in state or activity of a cell (in terms of movement, secretion, enzyme production, gene expression, etc.) as a result of an inositol stimulus. References: PMID:16496115 Sources: GOC:TermGenie